{
  "gene_symbol": "CHRNA2",
  "term_id": "GO:0035094",
  "gene": "UniProtKB:Q15822",
  "gene_name": "Neuronal acetylcholine receptor subunit alpha-2",
  "term_label": "response to nicotine"
}